{
  "term_label": "membrane",
  "gene_symbol": "DNAJC5",
  "term_id": "GO:0016020",
  "gene": "UniProtKB:Q9H3Z4",
  "gene_name": "DnaJ homolog subfamily C member 5"
}